positive regulation of keratinocyte proliferation [GO:0010838] (biological process) Relationships: is a type of regulation of keratinocyte proliferation [GO:0010837]; is a type of positive regulation of epithelial cell proliferation [GO:0050679]; positively regulates keratinocyte proliferation [GO:0043616] Definition: Any process that increases the rate, frequency or extent of keratinocyte proliferation. Keratinocyte proliferation is the multiplication or reproduction of keratinocytes, resulting in the expansion of a cell population. Sources: GOC:dph, GOC:tb